mesenchymal-epithelial cell signaling involved in prostate gland development [GO:0060739] (biological process) Definition: Any process that mediates the transfer of information from a mesenchymal cell to an epithelial cell where it is received and interpreted contributing to the progression of the prostate gland over time. Also known as: mesenchymal-epithelial cell signalling involved in prostate gland development Sources: GOC:dph Relationships: is a type of GO:0060638; is part of GO:0030850 Subtypes: GO:0060521